{
  "term_id": "GO:0003729",
  "gene_name": "Probable ATP-dependent RNA helicase DDX5",
  "term_label": "mRNA binding",
  "gene_symbol": "DDX5",
  "gene": "UniProtKB:P17844"
}